{
  "gene": "UniProtKB:Q9P2G1",
  "gene_symbol": "ANKIB1",
  "term_id": "GO:0000151",
  "gene_name": "Ankyrin repeat and IBR domain-containing protein 1",
  "term_label": "ubiquitin ligase complex"
}